{
  "gene": "UniProtKB:A0A8I5KYS1",
  "term_label": "Unknown cellular component",
  "gene_symbol": "A0A8I5KYS1",
  "term_id": "UNKNOWN:0003",
  "gene_name": "Vegetative cell wall protein gp1-like"
}